GDP binding [GO:0019003] (MF) Sources: GOC:ai Definition: Binding to GDP, guanosine 5'-diphosphate. Relationships: is a type of guanyl ribonucleotide binding [GO:0032561]; is a type of anion binding [GO:0043168] Regulation: negatively regulated by guanyl-nucleotide exchange factor activity [GO:0005085]; positively regulated by GDP-dissociation inhibitor activity [GO:0005092]